pinene catabolic process [GO:0033074] (biological process) Definition: The chemical reactions and pathways leading to the breakdown of the monoterpenoid pinene; alpha-pinene is (1S,5S)-2,6,6-trimethylbicyclo[3.1.1]hept-2-ene, and beta-pinene is (1S,5S)-6,6-dimethyl-2-methylenebicyclo[3.1.1]heptane. References: PMID:11452597 Sources: GOC:mah Also known as: pinene breakdown, pinene catabolism, pinene degradation Subtypes: GO:0046249 Relationships: is a type of pinene metabolic process [GO:0033073]; is a type of monoterpene catabolic process [GO:0043694]